{
  "gene_name": "Zinc finger protein 462",
  "term_label": "DNA-binding transcription factor activity",
  "gene": "UniProtKB:Q96JM2",
  "gene_symbol": "ZNF462",
  "term_id": "GO:0003700"
}